lipid transport involved in lipid storage [GO:0010877] (biological process) Sources: GOC:BHF, GOC:dph, GOC:tb Definition: The directed movement of lipids into cells that is part of their accumulation and maintenance. Relationships: is a type of lipid transport [GO:0006869]; BFO_0000050 lipid storage [GO:0019915] Subtypes: cholesterol transport involved in cholesterol storage [GO:0010879]